{
  "gene_symbol": "ARAP2",
  "gene": "UniProtKB:Q8WZ64",
  "term_id": "GO:0005096",
  "gene_name": "Arf-GAP with Rho-GAP domain, ANK repeat and PH domain-containing protein 2",
  "term_label": "GTPase activator activity"
}